{
  "term_id": "GO:0031543",
  "gene_name": "Prolyl 3-hydroxylase OGFOD1",
  "gene": "UniProtKB:Q8N543",
  "term_label": "peptidyl-proline dioxygenase activity",
  "gene_symbol": "OGFOD1"
}